{
  "gene_name": "POU domain, class 2, transcription factor 1",
  "gene_symbol": "POU2F1",
  "term_label": "DNA-binding transcription factor activity, RNA polymerase II-specific",
  "gene": "UniProtKB:P14859",
  "term_id": "GO:0000981"
}